{
  "gene": "UniProtKB:Q9UHV5",
  "gene_name": "Rap guanine nucleotide exchange factor-like 1",
  "gene_symbol": "RAPGEFL1",
  "term_label": "Rap protein signal transduction",
  "term_id": "GO:0032486"
}